{
  "gene_name": "Haloacid dehalogenase-like hydrolase domain-containing 5",
  "gene": "UniProtKB:Q9BXW7",
  "term_id": "UNKNOWN:0001",
  "term_label": "Unknown molecular function",
  "gene_symbol": "HDHD5"
}